{
  "term_label": "serotonin biosynthetic process",
  "gene_symbol": "TH",
  "gene_name": "Tyrosine 3-monooxygenase",
  "term_id": "GO:0042427",
  "gene": "UniProtKB:P07101"
}